positive regulation of interleukin-37 production [GO:0150139] (biological process) Relationships: is a type of positive regulation of cytokine production [GO:0001819]; is a type of regulation of interleukin-37 production [GO:0150136]; positively regulates interleukin-37 production [GO:0150137] Also known as: positive regulation of interleukin-37 biosynthetic process Definition: Any process that activates or increases the frequency, rate or extent of interleukin-37 production. Sources: GOC:aruk